astral microtubule depolymerization [GO:0060172] (biological process) Definition: The removal of tubulin heterodimers from one or both ends of an astral microtubule. An astral microtubule is any of the spindle microtubules that radiate in all directions from the spindle poles and are thought to contribute to the forces that separate the poles and position them in relation to the rest of the cell. Relationships: is a type of microtubule depolymerization [GO:0007019]; is a type of GO:0030953 Regulation: negatively regulated by negative regulation of astral microtubule depolymerization [GO:0032932] Sources: GOC:dph